{
  "gene_symbol": "ZNF22-AS1",
  "gene_name": "Uncharacterized protein ZNF22-AS1",
  "term_id": "UNKNOWN:0001",
  "gene": "UniProtKB:Q5T742",
  "term_label": "Unknown molecular function"
}